{
  "gene_symbol": "STAG3L3",
  "gene": "UniProtKB:P0CL85",
  "gene_name": "STAG3-like protein 3",
  "term_id": "UNKNOWN:0002",
  "term_label": "Unknown biological process"
}